regulation of protein localization to cell division site [GO:1901900] (biological process) Subtypes: regulation of protein localization to medial cortex [GO:0106011], regulation of protein localization to cell division site involved in mitotic actomyosin contractile ring assembly [GO:0110082], regulation of protein localization to cell division site involved in cytokinesis [GO:1901901], regulation of protein localization to cell division site involved in cell separation after cytokinesis [GO:1905391] Definition: Any process that modulates the frequency, rate or extent of protein localization to cell division site. Relationships: is a type of regulation of protein localization [GO:0032880]; regulates protein localization to cell division site [GO:0072741] Also known as: regulation of protein localisation to cell division site References: PMID:22573892 Sources: GOC:TermGenie, GOC:dph